{
  "gene_symbol": "RAD51B",
  "gene": "UniProtKB:O15315",
  "gene_name": "DNA repair protein RAD51 homolog 2",
  "term_id": "GO:0000400",
  "term_label": "four-way junction DNA binding"
}